proteasomal protein catabolic process [GO:0010498] (biological process) Subtypes: proteasomal ubiquitin-independent protein catabolic process [GO:0010499], GO:0036503, proteasome-mediated ubiquitin-dependent protein catabolic process [GO:0043161], EGAD pathway [GO:0140624] Sources: GOC:tb Also known as: proteasome-mediated protein catabolic process, proteasome-mediated protein catabolism Relationships: is_a protein catabolic process [GO:0030163]; is a type of GO:0051603 Definition: The chemical reactions and pathways resulting in the breakdown of a protein or peptide by hydrolysis of its peptide bonds that is mediated by the proteasome. Regulation: regulated by GO:0061136; RO_0002212 by negative regulation of proteasomal protein catabolic process [GO:1901799]; positively regulated by positive regulation of proteasomal protein catabolic process [GO:1901800]